{
  "gene_name": "SPRY domain-containing protein 4",
  "term_label": "Unknown biological process",
  "gene_symbol": "SPRYD4",
  "term_id": "UNKNOWN:0002",
  "gene": "UniProtKB:Q8WW59"
}